{
  "gene": "UniProtKB:Q5SVQ8",
  "gene_symbol": "ZBTB41",
  "term_id": "GO:0000981",
  "gene_name": "Zinc finger and BTB domain-containing protein 41",
  "term_label": "DNA-binding transcription factor activity, RNA polymerase II-specific"
}